cartilage development involved in endochondral bone morphogenesis [GO:0060351] (BP) Definition: The process whose specific outcome is the progression of the cartilage that will provide a scaffold for mineralization of endochondral bones. Relationships: is a type of GO:0051216; is part of GO:0060350 Subtypes: growth plate cartilage development [GO:0003417] Sources: GOC:dph